{
  "gene_name": "E3 ubiquitin-protein ligase MARCHF11",
  "term_label": "ubiquitin-protein transferase activity",
  "gene_symbol": "MARCHF11",
  "gene": "UniProtKB:A6NNE9",
  "term_id": "GO:0004842"
}